{
  "gene_name": "Androgen receptor",
  "term_id": "GO:0045944",
  "gene": "UniProtKB:P10275",
  "term_label": "positive regulation of transcription by RNA polymerase II",
  "gene_symbol": "AR"
}